GMP reductase complex [GO:1902560] (cellular component) Relationships: is a type of oxidoreductase complex [GO:1990204] References: PMID:12009299 Sources: GOC:TermGenie, GOC:bhm Note: An example of this is GMPR2 in human (UniProt Symbol Q9P2T1) in PMID:12009299 (inferred from direct assay). Definition: An oxidoreductase complex which is capable of GMP reductase activity. It catalyses the irreversible reaction: GMP + 2 H+ + NADPH => IMP + NADP+ + NH4. Also known as: GMP reductase, GMPR1 complex, GMPR2 complex, guanosine monophosphate reductase